{
  "gene_name": "Zinc finger protein 16",
  "gene": "UniProtKB:P17020",
  "term_id": "GO:0000981",
  "term_label": "DNA-binding transcription factor activity, RNA polymerase II-specific",
  "gene_symbol": "ZNF16"
}